{
  "term_label": "growth factor activity",
  "term_id": "GO:0008083",
  "gene": "UniProtKB:Q99075",
  "gene_name": "Proheparin-binding EGF-like growth factor",
  "gene_symbol": "HBEGF"
}